{
  "gene": "UniProtKB:Q9UJ98",
  "term_label": "chromatin",
  "gene_symbol": "STAG3",
  "term_id": "GO:0000785",
  "gene_name": "Cohesin subunit SA-3"
}